{
  "gene_name": "Fc receptor-like A",
  "term_label": "external side of plasma membrane",
  "gene": "UniProtKB:Q7L513",
  "term_id": "GO:0009897",
  "gene_symbol": "FCRLA"
}